{
  "gene": "UniProtKB:Q96G21",
  "gene_name": "U3 small nucleolar ribonucleoprotein protein IMP4",
  "term_id": "GO:0005730",
  "term_label": "nucleolus",
  "gene_symbol": "IMP4"
}